{
  "term_label": "regulation of telomere maintenance",
  "gene_name": "YLP motif-containing protein 1",
  "gene": "UniProtKB:P49750",
  "term_id": "GO:0032204",
  "gene_symbol": "YLPM1"
}